{
  "gene_symbol": "PHLDA3",
  "gene_name": "Pleckstrin homology-like domain family A member 3",
  "term_id": "UNKNOWN:0001",
  "gene": "UniProtKB:Q9Y5J5",
  "term_label": "Unknown molecular function"
}